{
  "term_id": "GO:0005886",
  "gene_name": "Alpha_beta hydrolase domain-containing protein 17B",
  "gene_symbol": "ABHD17B",
  "term_label": "plasma membrane",
  "gene": "UniProtKB:Q5VST6"
}